{
  "gene": "UniProtKB:P48357",
  "term_label": "cytokine receptor activity",
  "term_id": "GO:0004896",
  "gene_name": "Leptin receptor",
  "gene_symbol": "LEPR"
}